positive regulation of dopaminergic neuron differentiation [GO:1904340] (biological process) Relationships: is a type of positive regulation of neuron differentiation [GO:0045666]; is a type of regulation of dopaminergic neuron differentiation [GO:1904338]; positively regulates dopaminergic neuron differentiation [GO:0071542] Subtypes: positive regulation of midbrain dopaminergic neuron differentiation [GO:1904958] Also known as: up regulation of dopaminergic neuron differentiation, up-regulation of dopaminergic neuron differentiation, upregulation of dopaminergic neuron differentiation, activation of dopaminergic neuron differentiation Definition: Any process that activates or increases the frequency, rate or extent of dopaminergic neuron differentiation. References: PMID:15522889 Sources: GOC:TermGenie, GO_REF:0000058